{
  "term_label": "positive regulation of stress fiber assembly",
  "gene_symbol": "ARHGEF10",
  "term_id": "GO:0051496",
  "gene": "UniProtKB:O15013",
  "gene_name": "Rho guanine nucleotide exchange factor 10"
}